{
  "gene_name": "Ubiquitin carboxyl-terminal hydrolase 27",
  "term_label": "Unknown cellular component",
  "gene_symbol": "USP27X",
  "term_id": "UNKNOWN:0003",
  "gene": "UniProtKB:A6NNY8"
}